{
  "gene_symbol": "COL7A1",
  "gene_name": "Collagen alpha-1(VII) chain",
  "term_label": "basement membrane",
  "gene": "UniProtKB:Q02388",
  "term_id": "GO:0005604"
}